SAM complex [GO:0001401] (cellular component) Note: See also the cellular component term 'mitochondrial outer membrane translocase complex ; GO:0005742'. References: PMID:12891361 Also known as: TOB complex, mitochondrial sorting and assembly machinery complex Definition: A large complex of the mitochondrial outer membrane that mediates sorting of some imported proteins to the outer membrane and their assembly in the membrane; functions after import of incoming proteins by the mitochondrial outer membrane translocase complex. Relationships: is a type of mitochondrial outer membrane translocase complex [GO:0005742]